{
  "gene": "UniProtKB:Q96GP6",
  "term_label": "Unknown cellular component",
  "gene_symbol": "SCARF2",
  "term_id": "UNKNOWN:0003",
  "gene_name": "Scavenger receptor class F member 2"
}